peptidoglycan lytic transglycosylase activity [GO:0008933] (molecular function) Definition: Catalysis of the cleavage of a peptidoglycan chain into a peptidoglycan chain with N-acetyl-1,6-anhydromuramyl-[peptide] at the reducing end + a peptidoglycan chain with N-acetylglucosamine at the non-reducing end. Includes endolytic transglycosylase activity that fragments the glycan chain internally and exolytic transgylcosylase activity that cleaves a terminal disaccharide from the end of the glycan strand. Relationships: is a type of carbon-oxygen lyase activity, acting on polysaccharides [GO:0016837]; is a type of peptidoglycan muralytic activity [GO:0061783] References: PMID:10964424, PMID:22748813 Sources: EC:4.2.2.29 Subtypes: lytic endotransglycosylase activity [GO:0008932], GO:0140100 Also known as: lytic murein transglycosylase activity, lytic transglycosylase activity, murein transglycosylase activity